{
  "gene_symbol": "SF3B1",
  "gene": "UniProtKB:O75533",
  "term_id": "GO:0005689",
  "term_label": "U12-type spliceosomal complex",
  "gene_name": "Splicing factor 3B subunit 1"
}